inflammatory response to wounding [GO:0090594] (BP) Sources: GOC:add Definition: The immediate defensive reaction by vertebrate tissue to injury caused by chemical or physical agents. Regulation: regulated by regulation of inflammatory response to wounding [GO:0106014]; RO_0002212 by GO:0106015; RO_0002213 by GO:0106016 Relationships: is a type of inflammatory response [GO:0006954]; is_a response to wounding [GO:0009611]